{
  "term_id": "UNKNOWN:0003",
  "gene_symbol": "SHD",
  "gene": "UniProtKB:Q96IW2",
  "gene_name": "SH2 domain-containing adapter protein D",
  "term_label": "Unknown cellular component"
}